{
  "term_label": "Unknown cellular component",
  "gene": "UniProtKB:Q9H936",
  "gene_name": "Mitochondrial glutamate carrier 1",
  "gene_symbol": "SLC25A22",
  "term_id": "UNKNOWN:0003"
}